{
  "term_label": "endocytic vesicle",
  "term_id": "GO:0030139",
  "gene_name": "Signal transducing adapter molecule 2",
  "gene": "UniProtKB:O75886",
  "gene_symbol": "STAM2"
}